{
  "gene_symbol": "CD5L",
  "term_label": "regulation of complement activation",
  "term_id": "GO:0030449",
  "gene_name": "CD5 antigen-like",
  "gene": "UniProtKB:O43866"
}